{
  "gene": "UniProtKB:P57055",
  "gene_name": "Protein ripply3",
  "gene_symbol": "RIPPLY3",
  "term_label": "embryonic pattern specification",
  "term_id": "GO:0009880"
}